{
  "gene": "UniProtKB:Q8NBF1",
  "term_id": "GO:0006357",
  "gene_symbol": "GLIS1",
  "gene_name": "Zinc finger protein GLIS1",
  "term_label": "regulation of transcription by RNA polymerase II"
}